recognition of apoptotic cell [GO:0043654] (biological process) References: PMID:15536015 Sources: GOC:rk Relationships: is a type of GO:0006910; is part of GO:0043277 Also known as: detection of apoptotic cell, detection of apoptotic cell corpse, detection of cell corpse, recognition of apoptotic cell corpse, recognition of cell corpse Definition: The process in which a cell interprets signals (in the form of specific proteins and lipids) on the surface of a dying cell which it will engulf and remove by phagocytosis.